{
  "gene": "UniProtKB:P43354",
  "term_label": "cellular response to corticotropin-releasing hormone stimulus",
  "gene_symbol": "NR4A2",
  "gene_name": "Nuclear receptor subfamily 4 group A member 2",
  "term_id": "GO:0071376"
}